{
  "gene": "UniProtKB:A8K4G0",
  "gene_symbol": "CD300LB",
  "gene_name": "CMRF35-like molecule 7",
  "term_label": "transmembrane signaling receptor activity",
  "term_id": "GO:0004888"
}